collagen type XV trimer [GO:0005582] (cellular component) Definition: A collagen homotrimer of alpha1(XV) chains; a chondroitin sulfate proteoglycan often found in specialized basement membranes where it bridges between fibrils. References: PMID:11158616, PMID:11937714, PMID:21421911 Relationships: is a type of GO:0140156